{
  "term_id": "GO:0006886",
  "gene": "UniProtKB:P61764",
  "gene_symbol": "STXBP1",
  "gene_name": "Syntaxin-binding protein 1",
  "term_label": "intracellular protein transport"
}